dynein light intermediate chain binding [GO:0051959] (molecular function) Sources: GOC:bf Relationships: is a type of protein binding [GO:0005515] Definition: Binding to a light intermediate chain of the dynein complex.